regulation of corticotropin-releasing hormone secretion [GO:0043397] (biological process) Definition: Any process that modulates the frequency, rate or extent of corticotropin-releasing hormone secretion. References: PMID:11027914 Sources: GOC:go_curators Also known as: regulation of CRF secretion, regulation of CRH secretion, regulation of corticotropin-releasing factor secretion Relationships: is a type of regulation of peptide hormone secretion [GO:0090276]; regulates corticotropin-releasing hormone secretion [GO:0043396] Subtypes: negative regulation of corticotropin-releasing hormone secretion [GO:0051465], positive regulation of corticotropin-releasing hormone secretion [GO:0051466]